{
  "gene_symbol": "ALOXE3",
  "term_id": "UNKNOWN:0003",
  "gene": "UniProtKB:Q9BYJ1",
  "term_label": "Unknown cellular component",
  "gene_name": "Hydroperoxide isomerase ALOXE3"
}